{
  "term_label": "Golgi apparatus",
  "gene_symbol": "B4GALT2",
  "term_id": "GO:0005794",
  "gene": "UniProtKB:O60909",
  "gene_name": "Beta-1,4-galactosyltransferase 2"
}